{
  "term_id": "UNKNOWN:0001",
  "gene": "UniProtKB:Q5SR53",
  "term_label": "Unknown molecular function",
  "gene_name": "Putative uncharacterized protein PIK3CD-AS1",
  "gene_symbol": "PIK3CD-AS1"
}